{
  "term_id": "UNKNOWN:0001",
  "term_label": "Unknown molecular function",
  "gene_name": "T cell receptor beta variable 10-3",
  "gene_symbol": "TRBV10-3",
  "gene": "UniProtKB:A0A0K0K1G6"
}